{
  "gene": "UniProtKB:Q13639",
  "term_id": "GO:0051378",
  "term_label": "serotonin binding",
  "gene_symbol": "HTR4",
  "gene_name": "5-hydroxytryptamine receptor 4"
}